{
  "gene_name": "Refilin-A",
  "gene": "UniProtKB:Q6ZTI6",
  "term_id": "GO:0032432",
  "gene_symbol": "RFLNA",
  "term_label": "actin filament bundle"
}